anterograde dendritic transport [GO:0098937] (biological process) Subtypes: anterograde dendritic transport of messenger ribonucleoprotein complex [GO:0098964], anterograde dendritic transport of neurotransmitter receptor complex [GO:0098971], anterograde dendritic transport of mitochondrion [GO:0098972] Definition: The directed movement of organelles or molecules along microtubules from the cell body toward the postsynapse in dendrites. Sources: ISBN:0815316194 Relationships: is a type of dendritic transport [GO:0098935]; occurs in dendrite cytoplasm [GO:0032839]